{
  "term_id": "UNKNOWN:0002",
  "gene_symbol": "ERVK-16",
  "term_label": "Unknown biological process",
  "gene": "UniProtKB:P61578",
  "gene_name": "Endogenous retrovirus group K member 16 Rec protein"
}